{
  "term_label": "positive regulation of neuromuscular synaptic transmission",
  "gene_name": "43 kDa receptor-associated protein of the synapse",
  "term_id": "GO:1900075",
  "gene_symbol": "RAPSN",
  "gene": "UniProtKB:Q13702"
}